{
  "gene": "UniProtKB:Q6AI08",
  "gene_symbol": "HEATR6",
  "gene_name": "HEAT repeat-containing protein 6",
  "term_id": "UNKNOWN:0001",
  "term_label": "Unknown molecular function"
}